{
  "gene": "UniProtKB:Q7Z3H0",
  "term_label": "Unknown molecular function",
  "gene_name": "Photoreceptor ankyrin repeat protein",
  "term_id": "UNKNOWN:0001",
  "gene_symbol": "ANKRD33"
}